{
  "gene_name": "Serine protease inhibitor Kazal-type 5",
  "gene_symbol": "SPINK5",
  "gene": "UniProtKB:Q9NQ38",
  "term_label": "cell differentiation",
  "term_id": "GO:0030154"
}